{
  "term_label": "GTPase activity",
  "gene": "UniProtKB:P63000",
  "term_id": "GO:0003924",
  "gene_name": "Ras-related C3 botulinum toxin substrate 1",
  "gene_symbol": "RAC1"
}